{
  "term_id": "GO:0001676",
  "gene_name": "Long-chain-fatty-acid--CoA ligase 1",
  "gene": "UniProtKB:P33121",
  "term_label": "long-chain fatty acid metabolic process",
  "gene_symbol": "ACSL1"
}